{
  "term_id": "GO:0005829",
  "gene": "UniProtKB:P35558",
  "term_label": "cytosol",
  "gene_symbol": "PCK1",
  "gene_name": "Phosphoenolpyruvate carboxykinase, cytosolic [GTP]"
}